{
  "gene_symbol": "ZNHIT6",
  "term_id": "GO:0000463",
  "gene_name": "Box C_D snoRNA protein 1",
  "term_label": "maturation of LSU-rRNA from tricistronic rRNA transcript (SSU-rRNA, 5.8S rRNA, LSU-rRNA)",
  "gene": "UniProtKB:Q9NWK9"
}